thalian-diol desaturase activity [GO:0080004] (molecular function) Relationships: is a type of oxidoreductase activity, acting on paired donors, with incorporation or reduction of molecular oxygen [GO:0016705] Definition: Catalysis of the reaction: a thalian-diol = a desaturated thalian-diol. This reaction is the introduction of a double bond to a thalian-diol molecule at carbon 15. References: PMID:18356490